{
  "gene": "UniProtKB:Q8TBR5",
  "gene_name": "Putative uncharacterized protein CIRBP-AS1",
  "term_id": "UNKNOWN:0002",
  "gene_symbol": "CIRBP-AS1",
  "term_label": "Unknown biological process"
}